{
  "gene": "UniProtKB:Q92522",
  "term_id": "GO:0031492",
  "gene_name": "Histone H1.10",
  "term_label": "nucleosomal DNA binding",
  "gene_symbol": "H1-10"
}